zygotic determination of anterior/posterior axis, embryo [GO:0007354] (BP) Relationships: is a type of GO:0008595 Definition: The specification of the anterior/posterior axis of the embryo by products of genes expressed in the zygote; exemplified in insects by the gap genes, pair rule genes and segment polarity gene cascade. Sources: ISBN:0879694238, http://fly.ebi.ac.uk/allied-data/lk/interactive-fly/aimain/1aahome.htm